{
  "gene": "UniProtKB:Q8IXQ8",
  "term_id": "UNKNOWN:0003",
  "term_label": "Unknown cellular component",
  "gene_symbol": "PDZD9",
  "gene_name": "PDZ domain-containing protein 9"
}